response to 5-fluoro-2'-deoxyuridine [GO:0097330] (biological process) Definition: Any process that results in a change in state or activity of a cell or an organism (in terms of movement, secretion, enzyme production, gene expression, etc.) as a result of a 5-fluoro-2'-deoxyuridine stimulus. 5-fluoro-2'-deoxyuridine is a pyrimidine 2'-deoxyribonucleoside compound having 5-fluorouracil as the nucleobase; it is used to treat hepatic metastases of gastrointestinal adenocarcinomas and for palliation in malignant neoplasms of the liver and gastrointestinal tract. Sources: GOC:pr Relationships: is a type of GO:1901698; is a type of response to oxygen-containing compound [GO:1901700]